L-aspartate N-acetyltransferase activity [GO:0017188] (molecular function) Relationships: is_a L-amino-acid N-acetyltransferase activity [GO:0140085] Sources: RHEA:14165 Also known as: acetyl-CoA:L-aspartate N-acetyltransferase activity, aspartate N-acetyltransferase activity Definition: Catalysis of the reaction: L-aspartate + acetyl-CoA = N-acetyl-L-aspartate + CoA + H+.